{
  "gene_symbol": "RPRD1A",
  "term_label": "mRNA 3'-end processing",
  "gene": "UniProtKB:Q96P16",
  "term_id": "GO:0031124",
  "gene_name": "Regulation of nuclear pre-mRNA domain-containing protein 1A"
}